{
  "gene_symbol": "EIF4EBP3",
  "term_label": "negative regulation of translational initiation",
  "gene": "UniProtKB:O60516",
  "term_id": "GO:0045947",
  "gene_name": "Eukaryotic translation initiation factor 4E-binding protein 3"
}